{
  "gene_name": "Cation channel sperm-associated protein 3",
  "gene": "UniProtKB:Q86XQ3",
  "term_label": "acrosomal vesicle",
  "term_id": "GO:0001669",
  "gene_symbol": "CATSPER3"
}